{
  "gene": "UniProtKB:O00339",
  "gene_symbol": "MATN2",
  "gene_name": "Matrilin-2",
  "term_id": "UNKNOWN:0002",
  "term_label": "Unknown biological process"
}